VCP-NPL4-UFD1 AAA ATPase complex [GO:0034098] (CC) Definition: A multiprotein ATPase complex required for the efficient dislocation of ER-lumenal degradation substrates, and their subsequent proteolysis by the proteasome. In budding yeast, this complex includes Cdc48p, Npl4p and Ufd1p proteins. In mammals, this complex includes a hexamer of VCP/p97 (a cytosolic ATPase) and trimers of each of its cofactors UFD1L and NPL4 (NPLOC4) (e.g. a 6:3:3 stoichiometry). Relationships: is a type of GO:0098796; is a type of endoplasmic reticulum protein-containing complex [GO:0140534]; is part of endoplasmic reticulum membrane [GO:0005789]; has part GO:0036501 Also known as: p97-Ufd1-Npl4 complex, Cdc48p-Npl4p-Ufd1p AAA ATPase complex References: PMID:11813000, PMID:16179952